{
  "gene": "UniProtKB:P51149",
  "term_label": "late endosome",
  "gene_name": "Ras-related protein Rab-7a",
  "term_id": "GO:0005770",
  "gene_symbol": "RAB7A"
}